{
  "gene_symbol": "ZNF439",
  "gene": "UniProtKB:Q8NDP4",
  "term_label": "DNA-binding transcription factor activity, RNA polymerase II-specific",
  "gene_name": "Zinc finger protein 439",
  "term_id": "GO:0000981"
}